{
  "gene_symbol": "TLCD2",
  "term_id": "GO:0007009",
  "gene_name": "TLC domain-containing protein 2",
  "term_label": "plasma membrane organization",
  "gene": "UniProtKB:A6NGC4"
}